{
  "term_id": "GO:0043195",
  "term_label": "terminal bouton",
  "gene_symbol": "UNC13C",
  "gene_name": "Protein unc-13 homolog C",
  "gene": "UniProtKB:Q8NB66"
}